{
  "gene": "UniProtKB:O60518",
  "term_id": "GO:0008139",
  "term_label": "nuclear localization sequence binding",
  "gene_symbol": "RANBP6",
  "gene_name": "Ran-binding protein 6"
}